{
  "gene_name": "Serine_threonine-protein kinase ULK2",
  "term_id": "GO:0000045",
  "term_label": "autophagosome assembly",
  "gene": "UniProtKB:Q8IYT8",
  "gene_symbol": "ULK2"
}